{
  "term_id": "GO:0030018",
  "gene": "UniProtKB:O43707",
  "gene_symbol": "ACTN4",
  "gene_name": "Alpha-actinin-4",
  "term_label": "Z disc"
}